tonic skeletal muscle contraction [GO:0014720] (biological process) Sources: GOC:mtg_muscle Definition: A process in which force is generated within tonic skeletal muscle tissue, resulting in a change in muscle geometry. Force generation involves a chemo-mechanical energy conversion step that is carried out by the actin/myosin complex activity, which generates force through ATP hydrolysis. The tonic skeletal muscle is characterized by long lasting contractile responses and high resistance to fatigue. Regulation: regulated by GO:0014746; RO_0002213 by positive regulation of tonic skeletal muscle contraction [GO:0014747]; negatively regulated by negative regulation of tonic skeletal muscle contraction [GO:0014748] Relationships: is a type of GO:0003010